{
  "term_label": "chloride:bicarbonate antiporter activity",
  "gene_symbol": "SLC26A1",
  "gene_name": "Sulfate anion transporter 1",
  "term_id": "GO:0140900",
  "gene": "UniProtKB:Q9H2B4"
}